{
  "term_id": "GO:0005737",
  "term_label": "cytoplasm",
  "gene": "UniProtKB:Q9GZZ9",
  "gene_symbol": "UBA5",
  "gene_name": "Ubiquitin-like modifier-activating enzyme 5"
}